gap junction hemi-channel activity [GO:0055077] (molecular function) Also known as: connexon channel activity Definition: A wide pore channel activity that enables the transport of a solute across a membrane via a gap junction hemi-channel. Two gap junction hemi-channels coupled together form a complete gap junction. Relationships: is a type of wide pore channel activity [GO:0022829]; BFO_0000050 gap junction channel activity [GO:0005243] Sources: GOC:dgh